{
  "gene_symbol": "HSDL2",
  "gene": "UniProtKB:Q6YN16",
  "term_label": "Unknown molecular function",
  "gene_name": "Hydroxysteroid dehydrogenase-like protein 2",
  "term_id": "UNKNOWN:0001"
}